{
  "gene_name": "LYR motif-containing protein 1",
  "gene": "UniProtKB:O43325",
  "gene_symbol": "LYRM1",
  "term_label": "Unknown biological process",
  "term_id": "UNKNOWN:0002"
}